alpha5-beta1 integrin-LPP3 complex [GO:0071130] (CC) Definition: A protein complex that consists of an alpha5-beta1 integrin complex bound to lipid phosphate phosphohydrolase-3. References: PMID:16099422 Also known as: ITGA5-ITGB1-PPAP2B complex Relationships: is a type of plasma membrane protein complex [GO:0098797]